{
  "term_label": "Unknown biological process",
  "term_id": "UNKNOWN:0002",
  "gene": "UniProtKB:Q15170",
  "gene_symbol": "TCEAL1",
  "gene_name": "Transcription elongation factor A protein-like 1"
}